regulation of systemic arterial blood pressure by vasopressin [GO:0001992] (biological process) Definition: The regulation of blood pressure mediated by the signaling molecule vasopressin. Vasopressin is produced in the hypothalamus, and affects vasoconstriction, and renal water transport. Sources: GOC:mtg_cardio, ISBN:0721643949 Also known as: blood pressure regulation by vasopressin, vasopressin control of blood pressure Relationships: is_a regulation of systemic arterial blood pressure by hormone [GO:0001990]